positive regulation of hepatic stellate cell contraction [GO:0061874] (biological process) References: PMID:24204762 Definition: Any process that activates or increases the frequency, rate or extent of hepatic stellate cell contraction. Relationships: is a type of GO:0061873; is a type of positive regulation of actin filament-based movement [GO:1903116]; positively regulates hepatic stellate cell contraction [GO:0061872]